{
  "gene": "UniProtKB:Q14644",
  "gene_name": "Ras GTPase-activating protein 3",
  "gene_symbol": "RASA3",
  "term_label": "Unknown cellular component",
  "term_id": "UNKNOWN:0003"
}